{
  "gene": "UniProtKB:P56182",
  "gene_name": "Ribosomal RNA processing protein 1 homolog A",
  "term_id": "GO:0005694",
  "gene_symbol": "RRP1",
  "term_label": "chromosome"
}